{
  "gene_symbol": "TNFRSF11A",
  "gene": "UniProtKB:Q9Y6Q6",
  "term_label": "external side of plasma membrane",
  "gene_name": "Tumor necrosis factor receptor superfamily member 11A",
  "term_id": "GO:0009897"
}